{
  "term_label": "nucleus",
  "gene_symbol": "ZBTB40",
  "term_id": "GO:0005634",
  "gene_name": "Zinc finger and BTB domain-containing protein 40",
  "gene": "UniProtKB:Q9NUA8"
}